{
  "term_id": "GO:0005886",
  "gene_symbol": "SEMA6D",
  "gene": "UniProtKB:Q8NFY4",
  "gene_name": "Semaphorin-6D",
  "term_label": "plasma membrane"
}